{
  "gene": "UniProtKB:Q9UHY1",
  "gene_symbol": "NRBP1",
  "term_label": "cytosol",
  "gene_name": "Nuclear receptor-binding protein",
  "term_id": "GO:0005829"
}